{
  "gene_name": "Intraflagellar transport-associated protein",
  "term_id": "GO:0007283",
  "gene_symbol": "IFTAP",
  "gene": "UniProtKB:Q86VG3",
  "term_label": "spermatogenesis"
}